{
  "gene_name": "Lysine-specific demethylase 4D",
  "term_id": "GO:0000785",
  "term_label": "chromatin",
  "gene": "UniProtKB:Q6B0I6",
  "gene_symbol": "KDM4D"
}